{
  "gene": "UniProtKB:P37268",
  "term_id": "GO:0005789",
  "term_label": "endoplasmic reticulum membrane",
  "gene_name": "Squalene synthase",
  "gene_symbol": "FDFT1"
}